nuclear mineralocorticoid receptor binding [GO:0031962] (molecular function) References: PMID:12511169 Sources: GOC:mah Relationships: is a type of nuclear receptor binding [GO:0016922] Also known as: mineralocorticoid receptor binding Definition: Binding to a nuclear mineralocorticoid receptor.